{
  "gene_name": "Homeobox protein MIXL1",
  "term_label": "endoderm formation",
  "gene_symbol": "MIXL1",
  "term_id": "GO:0001706",
  "gene": "UniProtKB:Q9H2W2"
}